{
  "gene_symbol": "OR5A2",
  "term_label": "olfactory receptor activity",
  "gene": "UniProtKB:Q8NGI9",
  "term_id": "GO:0004984",
  "gene_name": "Olfactory receptor 5A2"
}